{
  "gene": "UniProtKB:P17661",
  "gene_name": "Desmin",
  "term_label": "sarcolemma",
  "gene_symbol": "DES",
  "term_id": "GO:0042383"
}